{
  "term_id": "UNKNOWN:0001",
  "gene_name": "Protein diaphanous homolog 3",
  "gene_symbol": "DIAPH3",
  "gene": "UniProtKB:Q9NSV4",
  "term_label": "Unknown molecular function"
}